{
  "gene_symbol": "PLXNA4",
  "gene_name": "Plexin-A4",
  "term_label": "axon guidance",
  "term_id": "GO:0007411",
  "gene": "UniProtKB:Q9HCM2"
}